{
  "term_label": "nucleus",
  "gene_name": "Z-DNA-binding protein 1",
  "term_id": "GO:0005634",
  "gene_symbol": "ZBP1",
  "gene": "UniProtKB:Q9H171"
}